regulation of toll-like receptor 6 signaling pathway [GO:0034151] (biological process) Subtypes: negative regulation of toll-like receptor 6 signaling pathway [GO:0034152], positive regulation of toll-like receptor 6 signaling pathway [GO:0034153] References: PMID:16551253, PMID:17328678 Sources: GOC:add Relationships: is a type of regulation of pattern recognition receptor signaling pathway [GO:0062207]; regulates toll-like receptor 6 signaling pathway [GO:0034150] Definition: Any process that modulates the frequency, rate, or extent of toll-like receptor 6 signaling pathway. Also known as: regulation of TLR6 signaling pathway, regulation of toll-like receptor 6 signalling pathway